{
  "term_label": "Unknown biological process",
  "gene_name": "Nuclear pore complex-interacting protein family member B8",
  "gene": "UniProtKB:E9PQR5",
  "gene_symbol": "NPIPB8",
  "term_id": "UNKNOWN:0002"
}